sensory perception of bitter taste [GO:0050913] (biological process) Sources: GOC:ai Definition: The series of events required to receive a bitter taste stimulus, convert it to a molecular signal, and recognize and characterize the signal. This is a neurological process. Regulation: regulated by regulation of sensory perception of bitter taste [GO:1904660]; negatively regulated by negative regulation of sensory perception of bitter taste [GO:1904661]; positively regulated by GO:1904662 Relationships: is a type of sensory perception of taste [GO:0050909] Also known as: bitter taste perception